{
  "term_id": "UNKNOWN:0002",
  "gene_name": "Chromatin complexes subunit BAP18",
  "gene_symbol": "BAP18",
  "term_label": "Unknown biological process",
  "gene": "UniProtKB:Q8IXM2"
}